{
  "gene": "UniProtKB:Q9GZK6",
  "term_label": "detection of chemical stimulus involved in sensory perception of smell",
  "term_id": "GO:0050911",
  "gene_name": "Olfactory receptor 2J1",
  "gene_symbol": "OR2J1"
}